protein K11-linked ubiquitination [GO:0070979] (BP) References: PMID:18485873, PMID:20655260, PMID:21113135 Sources: GOC:jsg, GOC:pr, GOC:sp Definition: A protein ubiquitination process in which ubiquitin monomers are attached to a protein, and then ubiquitin polymers are formed by linkages between lysine residues at position 11 of the ubiquitin monomers. K11-linked polyubiquitination targets the substrate protein for degradation. The anaphase-promoting complex promotes the degradation of mitotic regulators by assembling K11-linked polyubiquitin chains. Relationships: is a type of protein polyubiquitination [GO:0000209]